{
  "term_id": "GO:0005615",
  "gene": "UniProtKB:Q99877",
  "gene_name": "Histone H2B type 1-N",
  "gene_symbol": "H2BC15",
  "term_label": "extracellular space"
}